{
  "gene_symbol": "BAX",
  "gene_name": "Apoptosis regulator BAX",
  "term_id": "GO:0001836",
  "term_label": "release of cytochrome c from mitochondria",
  "gene": "UniProtKB:Q07812"
}